{
  "term_label": "RNA 7-methylguanosine cap binding",
  "gene_name": "m7GpppX diphosphatase",
  "term_id": "GO:0000340",
  "gene": "UniProtKB:Q96C86",
  "gene_symbol": "DCPS"
}